negative regulation of lung goblet cell differentiation [GO:1901250] (biological process) Definition: Any process that stops, prevents or reduces the frequency, rate or extent of lung goblet cell differentiation. Relationships: is a type of negative regulation of epithelial cell differentiation [GO:0030857]; is a type of negative regulation of multicellular organismal process [GO:0051241]; is a type of GO:1901249; negatively regulates lung goblet cell differentiation [GO:0060480] Sources: GOC:BHF, GOC:TermGenie Also known as: down regulation of lung goblet cell differentiation, down regulation of pulmonary goblet cell differentiation, down-regulation of lung goblet cell differentiation, down-regulation of pulmonary goblet cell differentiation, downregulation of lung goblet cell differentiation, downregulation of pulmonary goblet cell differentiation, negative regulation of pulmonary goblet cell differentiation, inhibition of lung goblet cell differentiation, inhibition of pulmonary goblet cell differentiation